{
  "gene_name": "Protein MAK16 homolog",
  "gene_symbol": "MAK16",
  "term_id": "GO:0030687",
  "gene": "UniProtKB:Q9BXY0",
  "term_label": "preribosome, large subunit precursor"
}